NuA4 histone acetyltransferase complex binding [GO:0062060] (molecular function) Relationships: is a type of protein-containing complex binding [GO:0044877] Definition: Binding to a NuA4 histone acetyltransferase complex. References: PMID:15528408